{
  "term_id": "GO:0005763",
  "term_label": "mitochondrial small ribosomal subunit",
  "gene_symbol": "MRPS17",
  "gene_name": "Small ribosomal subunit protein uS17m",
  "gene": "UniProtKB:Q9Y2R5"
}